{
  "gene_symbol": "UBE2Q1",
  "term_id": "GO:0000209",
  "term_label": "protein polyubiquitination",
  "gene_name": "Ubiquitin-conjugating enzyme E2 Q1",
  "gene": "UniProtKB:Q7Z7E8"
}